{
  "gene_name": "HLA class II histocompatibility antigen, DM alpha chain",
  "term_label": "MHC class II protein complex",
  "gene_symbol": "HLA-DMA",
  "gene": "UniProtKB:P28067",
  "term_id": "GO:0042613"
}